{
  "gene_name": "Putative uncharacterized protein TXNRD3NB",
  "term_id": "UNKNOWN:0003",
  "term_label": "Unknown cellular component",
  "gene": "UniProtKB:Q6F5E7",
  "gene_symbol": "TXNRD3NB"
}